{
  "gene_name": "Macrophage-capping protein",
  "gene": "UniProtKB:P40121",
  "term_label": "actin filament severing",
  "term_id": "GO:0051014",
  "gene_symbol": "CAPG"
}